{
  "gene_name": "Ribosomal protein uL3-like",
  "term_id": "GO:0006412",
  "gene_symbol": "RPL3L",
  "term_label": "translation",
  "gene": "UniProtKB:Q92901"
}